metanephric capsule specification [GO:0072267] (biological process) Sources: GOC:mtg_kidney_jan10 Relationships: is a type of GO:0072130; is a type of pattern specification involved in metanephros development [GO:0072268]; is part of GO:0072266 Definition: The regionalization process in which the identity of the metanephric capsule is specified. Identity is considered to be the aggregate of characteristics by which a structure is recognized.